renal artery morphogenesis [GO:0061441] (BP) Definition: The process in which the anatomical structure of a renal artery is generated and organized. Renal arteries supply the kidneys with blood. Relationships: is a type of artery morphogenesis [GO:0048844]; is part of kidney vasculature morphogenesis [GO:0061439] References: PMID:11891195 Sources: GOC:mtg_kidney_jan10